{
  "term_label": "Unknown molecular function",
  "term_id": "UNKNOWN:0001",
  "gene_symbol": "FLNB",
  "gene_name": "Filamin-B",
  "gene": "UniProtKB:O75369"
}